{
  "gene_name": "Josephin-2",
  "term_label": "Unknown biological process",
  "gene_symbol": "JOSD2",
  "gene": "UniProtKB:Q8TAC2",
  "term_id": "UNKNOWN:0002"
}